{
  "term_id": "GO:0000981",
  "gene": "UniProtKB:P0CJ89",
  "term_label": "DNA-binding transcription factor activity, RNA polymerase II-specific",
  "gene_name": "Double homeobox protein 4-like protein 6",
  "gene_symbol": "DUX4L6"
}